{
  "gene_name": "Forkhead box protein D4-like 5",
  "gene_symbol": "FOXD4L5",
  "term_label": "cell differentiation",
  "term_id": "GO:0030154",
  "gene": "UniProtKB:Q5VV16"
}